3-methyl-2-oxobutanoate dehydrogenase (ferredoxin) activity [GO:0043807] (molecular function) Definition: Catalysis of the reaction: 3-methyl-2-oxobutanoate + CoA + oxidized ferredoxin = S-(2-methylpropanoyl)-CoA + CO2 + reduced ferredoxin. Sources: EC:1.2.7.7 Also known as: 3-methyl-2-oxobutanoate:ferredoxin oxidoreductase (decarboxylating; CoA-2-methylpropanoylating), 2-ketoisovalerate ferredoxin reductase activity, 2-oxoisovalerate ferredoxin reductase activity, 3-methyl-2-oxobutanoate synthase (ferredoxin) activity, VOR, branched-chain ketoacid ferredoxin reductase activity, branched-chain oxo acid ferredoxin reductase activity, keto-valine-ferredoxin oxidoreductase activity, ketoisovalerate ferredoxin reductase activity, ketoisovalerate oxidoreductase activity Relationships: is a type of oxidoreductase activity, acting on the aldehyde or oxo group of donors, iron-sulfur protein as acceptor [GO:0016625]